{
  "term_id": "UNKNOWN:0001",
  "term_label": "Unknown molecular function",
  "gene_symbol": "PHB2",
  "gene_name": "Prohibitin-2",
  "gene": "UniProtKB:Q99623"
}